{
  "gene_name": "T cell receptor gamma joining P1 (Fragment)",
  "term_id": "UNKNOWN:0001",
  "gene_symbol": "TRGJP1",
  "gene": "UniProtKB:A0A0A0MT97",
  "term_label": "Unknown molecular function"
}